{
  "gene": "UniProtKB:Q9NQX0",
  "term_id": "UNKNOWN:0001",
  "term_label": "Unknown molecular function",
  "gene_symbol": "PRDM6",
  "gene_name": "Putative histone-lysine N-methyltransferase PRDM6"
}